{
  "gene_symbol": "UBR2",
  "term_label": "ubiquitin ligase complex",
  "gene_name": "E3 ubiquitin-protein ligase UBR2",
  "gene": "UniProtKB:Q8IWV8",
  "term_id": "GO:0000151"
}